{
  "gene_name": "Coiled-coil domain-containing protein 146",
  "gene_symbol": "CCDC146",
  "term_id": "UNKNOWN:0001",
  "term_label": "Unknown molecular function",
  "gene": "UniProtKB:Q8IYE0"
}